{
  "term_label": "cytoplasm",
  "gene": "UniProtKB:P61328",
  "term_id": "GO:0005737",
  "gene_name": "Fibroblast growth factor 12",
  "gene_symbol": "FGF12"
}